{
  "gene_name": "Zonadhesin",
  "gene_symbol": "ZAN",
  "gene": "UniProtKB:Q9Y493",
  "term_label": "Unknown biological process",
  "term_id": "UNKNOWN:0002"
}